{
  "gene": "UniProtKB:Q9NWU5",
  "term_label": "structural constituent of ribosome",
  "gene_name": "Large ribosomal subunit protein uL22m",
  "term_id": "GO:0003735",
  "gene_symbol": "MRPL22"
}